{
  "gene_symbol": "ZNF525",
  "term_id": "GO:0003700",
  "gene": "UniProtKB:Q8N782",
  "gene_name": "Zinc finger protein 525",
  "term_label": "DNA-binding transcription factor activity"
}